{
  "gene_name": "Activity-dependent neuroprotector homeobox protein",
  "gene_symbol": "ADNP",
  "gene": "UniProtKB:Q9H2P0",
  "term_label": "Unknown molecular function",
  "term_id": "UNKNOWN:0001"
}